{
  "term_label": "signal transduction",
  "gene_symbol": "PTPRU",
  "term_id": "GO:0007165",
  "gene": "UniProtKB:Q92729",
  "gene_name": "Receptor-type tyrosine-protein phosphatase U"
}